BRCA1-BARD1 complex [GO:0031436] (CC) Definition: A heterodimeric complex comprising BRCA1 and BARD1, which possesses ubiquitin ligase activity and is involved in genome maintenance, possibly by functioning in surveillance for DNA damage. References: PMID:12787778 Relationships: is a type of nuclear ubiquitin ligase complex [GO:0000152]